1-penten-3-one reductase activity [GO:0102235] (MF) Sources: GOC:pz Definition: Catalysis of the reaction: 1-penten-3-one + NADPH + H+ = 1-pentan-3-one + NADP. Relationships: is a type of oxidoreductase activity, acting on the CH-CH group of donors, NAD or NADP as acceptor [GO:0016628]